{
  "gene": "UniProtKB:Q9BR76",
  "gene_symbol": "CORO1B",
  "term_label": "plasma membrane",
  "gene_name": "Coronin-1B",
  "term_id": "GO:0005886"
}